phosphate:proton symporter activity [GO:0015317] (molecular function) Definition: Enables the transfer of a solute or solutes from one side of a membrane to the other according to the reaction: phosphate(out) + H+(out) = phosphate(in) + H+(in). Sources: TC:2.A.1.9.- Also known as: phosphate ion carrier activity, phosphate:hydrogen symporter activity Relationships: is a type of solute:proton symporter activity [GO:0015295]